{
  "gene": "UniProtKB:Q9HCG7",
  "term_label": "Unknown cellular component",
  "term_id": "UNKNOWN:0003",
  "gene_symbol": "GBA2",
  "gene_name": "Non-lysosomal glucosylceramidase"
}